biphenyl-2,3-diol 1,2-dioxygenase activity [GO:0018583] (molecular function) Sources: EC:1.13.11.39 Relationships: is a type of GO:0016702 Definition: Catalysis of the reaction: biphenyl-2,3-diol + O2 = 2-hydroxy-6-oxo-6-phenylhexa-2,4-dienoate + H2O. Also known as: 2,3-dihydroxybiphenyl 1,2-dioxygenase activity, 2,3-dihydroxybiphenyl dioxygenase activity, biphenyl-2,3-diol dioxygenase activity, biphenyl-2,3-diol:oxygen 1,2-oxidoreductase (decyclizing)